clathrin coat of coated pit [GO:0030132] (cellular component) Definition: The coat found on coated pits and the coated vesicles derived from coated pits; comprises clathrin and the AP-2 adaptor complex. Sources: GOC:mah Relationships: is a type of GO:0030118; is a type of plasma membrane protein complex [GO:0098797]; is part of clathrin-coated pit [GO:0005905]